{
  "gene": "UniProtKB:Q96PR1",
  "term_label": "potassium ion transmembrane transport",
  "term_id": "GO:0071805",
  "gene_symbol": "KCNC2",
  "gene_name": "Potassium voltage-gated channel subfamily C member 2"
}